{
  "term_label": "inflammatory response",
  "term_id": "GO:0006954",
  "gene": "UniProtKB:P43115",
  "gene_symbol": "PTGER3",
  "gene_name": "Prostaglandin E2 receptor EP3 subtype"
}